positive regulation of translational termination [GO:0045905] (biological process) Sources: GOC:go_curators Also known as: up regulation of translational termination, up-regulation of translational termination, upregulation of translational termination, activation of translational termination, stimulation of translational termination Definition: Any process that activates or increases the frequency, rate or extent of translational termination. Relationships: is a type of regulation of translational termination [GO:0006449]; is a type of positive regulation of protein-containing complex disassembly [GO:0043243]; is a type of positive regulation of translation [GO:0045727]; positively regulates translational termination [GO:0006415]